{
  "term_label": "nucleoplasm",
  "gene": "UniProtKB:O43684",
  "gene_name": "Mitotic checkpoint protein BUB3",
  "gene_symbol": "BUB3",
  "term_id": "GO:0005654"
}